peptide-O-fucosyltransferase activity [GO:0046922] (molecular function) Relationships: is a type of fucosyltransferase activity [GO:0008417]; is a type of catalytic activity, acting on a protein [GO:0140096]; is part of protein O-linked glycosylation via fucose [GO:0036066] Also known as: GDP-L-fucose:polypeptide fucosyltransferase activity, GDP-beta-L-fucose:polypeptide O-alpha-L-fucosyltransferase activity, GDP-fucose protein O-fucosyltransferase activity, GDP-fucose:polypeptide fucosyltransferase activity Definition: Catalysis of the transfer of an alpha-L-fucosyl residue from GDP-beta-L-fucose to the serine hydroxy group of a protein acceptor. Sources: EC:2.4.1.221